{
  "gene_symbol": "AR",
  "gene_name": "Androgen receptor",
  "term_id": "GO:0004879",
  "term_label": "nuclear receptor activity",
  "gene": "UniProtKB:P10275"
}